{
  "gene": "UniProtKB:Q9BZF9",
  "gene_name": "Uveal autoantigen with coiled-coil domains and ankyrin repeats",
  "gene_symbol": "UACA",
  "term_label": "intrinsic apoptotic signaling pathway in response to DNA damage",
  "term_id": "GO:0008630"
}